lipoprotein particle receptor activity [GO:0030228] (molecular function) References: PMID:12827279 Sources: GOC:bf, GOC:mah Also known as: lipoprotein receptor activity, plasma lipoprotein particle receptor activity Relationships: is a type of cargo receptor activity [GO:0038024]; has part lipoprotein particle binding [GO:0071813] Subtypes: low-density lipoprotein particle receptor activity [GO:0005041], very-low-density lipoprotein particle receptor activity [GO:0030229], high-density lipoprotein particle receptor activity [GO:0070506], oxidised low-density lipoprotein particle receptor activity [GO:0150025] Definition: Combining with a lipoprotein particle and delivering the lipoprotein particle into the cell via endocytosis. A lipoprotein particle, also known as a lipoprotein, is a clathrate complex consisting of a lipid enwrapped in a protein host without covalent binding in such a way that the complex has a hydrophilic outer surface consisting of all the protein and the polar ends of any phospholipids. Note: This term is intended for cell surface receptors that bind and internalize a lipoprotein particle. For members of the lipoprotein receptor family that transduce a signal rather than endocytose their ligand, consider instead the terms 'signaling receptor activity ; GO:0038023' and its children, or 'reelin receptor activity ; GO:0038025'.